{
  "term_id": "GO:0002218",
  "gene_name": "Myeloid cell nuclear differentiation antigen",
  "gene_symbol": "MNDA",
  "gene": "UniProtKB:P41218",
  "term_label": "activation of innate immune response"
}